{
  "gene": "UniProtKB:Q70EL3",
  "gene_name": "Inactive ubiquitin carboxyl-terminal hydrolase 50",
  "term_id": "GO:0014069",
  "gene_symbol": "USP50",
  "term_label": "postsynaptic density"
}